{
  "term_id": "GO:0045294",
  "gene": "UniProtKB:P18206",
  "gene_name": "Vinculin",
  "gene_symbol": "VCL",
  "term_label": "alpha-catenin binding"
}